enteroendocrine cell differentiation [GO:0035883] (biological process) Relationships: is a type of GO:0030855 Sources: CL:0000164, GOC:bf Definition: The process in which a relatively unspecialized cell acquires specialized structural and/or functional features of an enteroendocrine cell. Enteroendocrine cells are hormonally active epithelial cells in the gut that constitute the diffuse neuroendocrine system. Subtypes: type B pancreatic cell differentiation [GO:0003309], GO:0003310, pancreatic D cell differentiation [GO:0003311], pancreatic PP cell differentiation [GO:0003312], stomach neuroendocrine cell differentiation [GO:0061102], GO:0090104